{
  "term_id": "UNKNOWN:0003",
  "term_label": "Unknown cellular component",
  "gene_name": "Gamma-crystallin C",
  "gene": "UniProtKB:P07315",
  "gene_symbol": "CRYGC"
}